{
  "term_id": "GO:0000981",
  "gene_symbol": "ZFP69B",
  "term_label": "DNA-binding transcription factor activity, RNA polymerase II-specific",
  "gene_name": "Zinc finger protein 69 homolog B",
  "gene": "UniProtKB:Q9UJL9"
}